{
  "gene": "UniProtKB:O60603",
  "gene_symbol": "TLR2",
  "term_label": "receptor complex",
  "term_id": "GO:0043235",
  "gene_name": "Toll-like receptor 2"
}